{
  "gene": "UniProtKB:Q96RG2",
  "gene_symbol": "PASK",
  "term_label": "protein serine/threonine kinase activity",
  "term_id": "GO:0004674",
  "gene_name": "PAS domain-containing serine_threonine-protein kinase"
}